{
  "gene": "UniProtKB:Q96J86",
  "gene_name": "Cysteine and tyrosine-rich protein 1",
  "term_label": "Unknown biological process",
  "gene_symbol": "CYYR1",
  "term_id": "UNKNOWN:0002"
}